{
  "gene_name": "Collagen alpha-1(XVI) chain",
  "term_label": "extracellular matrix organization",
  "term_id": "GO:0030198",
  "gene_symbol": "COL16A1",
  "gene": "UniProtKB:Q07092"
}